{
  "term_id": "UNKNOWN:0001",
  "gene": "UniProtKB:Q8IVF2",
  "gene_symbol": "AHNAK2",
  "gene_name": "Protein AHNAK2",
  "term_label": "Unknown molecular function"
}